alditol phosphate metabolic process [GO:0052646] (biological process) Also known as: alditol phosphate metabolism References: PMID:30240188 Relationships: is a type of phosphate-containing compound metabolic process [GO:0006796]; is a type of GO:0019637; is a type of carbohydrate derivative metabolic process [GO:1901135] Definition: The chemical reactions and pathways involving alditol phosphates, any phosphorylated polyhydric alcohol derived from the acyclic form of a monosaccharide by reduction of its aldehyde or keto group to an alcoholic group. Subtypes: glycerol-3-phosphate metabolic process [GO:0006072], F420-0 metabolic process [GO:0052645], coenzyme gamma-F420-2 biosynthetic process [GO:2001121], lysobisphosphatidic acid metabolic process [GO:2001311]